fatty alcohol catabolic process [GO:1903174] (biological process) Subtypes: octanol catabolic process [GO:0046172] References: PMID:24036493 Sources: GOC:TermGenie, GOC:mengo_curators, GO_REF:0000068 Also known as: fatty alcohol breakdown, fatty alcohol catabolism, fatty alcohol degradation Relationships: is a type of GO:0046164; is a type of fatty acid derivative catabolic process [GO:1901569]; is a type of GO:1903173 Definition: The chemical reactions and pathways resulting in the breakdown of fatty alcohol.